thromboxane receptor activity [GO:0004960] (molecular function) Definition: Combining with a thromboxane (TXA) to initiate a change in cell activity. Sources: ISBN:0198506732 Also known as: TXA receptor activity Relationships: is_a GO:0004954 Subtypes: thromboxane A2 receptor activity [GO:0004961]